{
  "term_label": "DNA damage response",
  "term_id": "GO:0006974",
  "gene": "UniProtKB:Q9H993",
  "gene_symbol": "ARMT1",
  "gene_name": "Damage-control phosphatase ARMT1"
}